regulation of neutrophil chemotaxis [GO:0090022] (biological process) Relationships: is a type of GO:0071622; is_a GO:1902622; regulates neutrophil chemotaxis [GO:0030593] Definition: Any process that modulates the frequency, rate, or extent of neutrophil chemotaxis. Neutrophil chemotaxis is the directed movement of a neutrophil cell, the most numerous polymorphonuclear leukocyte found in the blood, in response to an external stimulus, usually an infection or wounding. Sources: GOC:dph, GOC:tb Subtypes: positive regulation of neutrophil chemotaxis [GO:0090023], GO:0090024